1-(5-phosphoribosyl)-5-[(5-phosphoribosylamino)methylideneamino]imidazole-4-carboxamide isomerase activity [GO:0003949] (MF) Definition: Catalysis of the reaction: 1-(5-phosphoribosyl)-5-[(5-phosphoribosylamino)methylideneamino]imidazole-4-carboxamide = 5-[(5-phospho-1-deoxy-D-ribulos-1-ylimino)methylamino]-1-(5-phospho-D-ribosyl)imidazole-4-carboxamide. Relationships: is a type of intramolecular oxidoreductase activity, interconverting aldoses and ketoses [GO:0016861] Sources: EC:5.3.1.16, RHEA:15469 Also known as: 1-(5-phosphoribosyl)-5-[(5-phosphoribosylamino)methylideneamino]imidazole-4-carboxamide aldose-ketose-isomerase activity, 1-(5-phosphoribosyl)-5-[(5-phosphoribosylamino)methylideneamino]imidazole-4-carboxamide ketol-isomerase activity, N-(5'-phospho-D-ribosylformimino)-5-amino-1-(5''-phosphoribosyl)-4-imidazolecarboxamide isomerase activity, N-(phosphoribosylformimino) aminophosphoribosylimidazolecarboxamide isomerase activity, phosphoribosylformimino-5-aminoimidazole carboxamide ribotide isomerase activity, phosphoribosylformiminoaminophosphoribosylimidazolecarboxamide isomerase activity